{
  "gene_name": "Myosin light chain 1_3, skeletal muscle isoform",
  "gene_symbol": "MYL1",
  "gene": "UniProtKB:P05976",
  "term_id": "UNKNOWN:0002",
  "term_label": "Unknown biological process"
}